{
  "gene_symbol": "DYDC1",
  "term_label": "radial spoke",
  "gene": "UniProtKB:Q8WWB3",
  "gene_name": "DPY30 domain-containing protein 1",
  "term_id": "GO:0001534"
}